{
  "gene_symbol": "NECAB1",
  "gene": "UniProtKB:Q8N987",
  "gene_name": "N-terminal EF-hand calcium-binding protein 1",
  "term_label": "regulation of amyloid precursor protein biosynthetic process",
  "term_id": "GO:0042984"
}